cytosine deaminase activity [GO:0004131] (molecular function) Relationships: is a type of hydrolase activity, acting on carbon-nitrogen (but not peptide) bonds, in cyclic amidines [GO:0016814]; is a type of deaminase activity [GO:0019239] Also known as: cytosine aminohydrolase activity, isocytosine deaminase activity Definition: Catalysis of the reaction: cytosine + H2O = uracil + NH3. Sources: EC:3.5.4.1